{
  "term_label": "beta-1,3-galactosyl-O-glycosyl-glycoprotein beta-1,6-N-acetylglucosaminyltransferase activity",
  "gene": "UniProtKB:Q02742",
  "term_id": "GO:0003829",
  "gene_name": "Beta-1,3-galactosyl-O-glycosyl-glycoprotein beta-1,6-N-acetylglucosaminyltransferase",
  "gene_symbol": "GCNT1"
}